{
  "gene": "UniProtKB:Q16890",
  "term_label": "positive regulation of JNK cascade",
  "term_id": "GO:0046330",
  "gene_symbol": "TPD52L1",
  "gene_name": "Tumor protein D53"
}